{
  "term_id": "GO:0070006",
  "gene": "UniProtKB:Q07075",
  "gene_symbol": "ENPEP",
  "term_label": "metalloaminopeptidase activity",
  "gene_name": "Glutamyl aminopeptidase"
}